{
  "term_label": "thrombopoietin-mediated signaling pathway",
  "gene_symbol": "SH2B3",
  "gene": "UniProtKB:Q9UQQ2",
  "gene_name": "SH2B adapter protein 3",
  "term_id": "GO:0038163"
}